pyruvate import into mitochondria [GO:0006850] (biological process) Relationships: is a type of GO:0170036; is a type of pyruvate transmembrane transport [GO:1901475] References: PMID:22628558 Sources: GOC:vw Also known as: mitochondrial pyruvate transport, pyruvate membrane transport in mitochondria, pyruvate membrane transport in mitochondrion, pyruvate transmembrane transport in mitochondria, pyruvate transmembrane transport in mitochondrion Definition: The process in which pyruvate is transported from the cytosol into the mitochondrial matrix.